CCR10 chemokine receptor binding [GO:0031735] (molecular function) Relationships: is a type of CCR chemokine receptor binding [GO:0048020] Sources: GOC:mah, GOC:nln Also known as: CCR10 chemokine receptor ligand Definition: Binding to a CCR10 chemokine receptor.